calcium-dependent protein serine/threonine kinase activity [GO:0009931] (molecular function) Subtypes: calcium,diacylglycerol-dependent serine/threonine kinase activity [GO:0004698] Sources: GOC:mah Definition: Calcium-dependent catalysis of the reactions: ATP + a protein serine = ADP + protein serine phosphate; and ATP + a protein threonine = ADP + protein threonine phosphate. Relationships: is a type of protein serine/threonine kinase activity [GO:0004674] Regulation: negatively regulated by calcium-dependent protein kinase inhibitor activity [GO:0008427]; regulated by GO:0010858